{
  "term_id": "GO:0003097",
  "gene_name": "Aquaporin-1",
  "term_label": "renal water transport",
  "gene_symbol": "AQP1",
  "gene": "UniProtKB:P29972"
}